{
  "term_label": "recycling endosome membrane",
  "term_id": "GO:0055038",
  "gene_symbol": "SCAMP2",
  "gene_name": "Secretory carrier-associated membrane protein 2",
  "gene": "UniProtKB:O15127"
}